negative regulation of fat cell proliferation [GO:0070345] (biological process) Also known as: down regulation of fat cell proliferation, down-regulation of fat cell proliferation, downregulation of fat cell proliferation, negative regulation of adipocyte proliferation, negative regulation of adipose cell proliferation, inhibition of fat cell proliferation Definition: Any process that stops or decreases the rate or extent of fat cell proliferation. Sources: GOC:mah, GOC:sl Relationships: is a type of negative regulation of cell population proliferation [GO:0008285]; is a type of regulation of fat cell proliferation [GO:0070344]; negatively regulates GO:0070341 Subtypes: GO:0070348, GO:0070351